{
  "gene_name": "BRCA2 and CDKN1A-interacting protein",
  "term_label": "Unknown molecular function",
  "gene_symbol": "BCCIP",
  "term_id": "UNKNOWN:0001",
  "gene": "UniProtKB:Q9P287"
}